{
  "term_label": "Golgi to vacuole transport",
  "term_id": "GO:0006896",
  "gene_symbol": "AP1G2",
  "gene": "UniProtKB:O75843",
  "gene_name": "AP-1 complex subunit gamma-like 2"
}